{
  "gene_name": "Sideroflexin-1",
  "term_label": "transmembrane transporter activity",
  "gene_symbol": "SFXN1",
  "gene": "UniProtKB:Q9H9B4",
  "term_id": "GO:0022857"
}